{
  "term_label": "maturation of LSU-rRNA from tricistronic rRNA transcript (SSU-rRNA, 5.8S rRNA, LSU-rRNA)",
  "term_id": "GO:0000463",
  "gene": "UniProtKB:Q9H7B2",
  "gene_name": "Ribosome production factor 2 homolog",
  "gene_symbol": "RPF2"
}